{
  "term_id": "GO:0005856",
  "gene": "UniProtKB:Q8IYE0",
  "term_label": "cytoskeleton",
  "gene_symbol": "CCDC146",
  "gene_name": "Coiled-coil domain-containing protein 146"
}